{
  "gene_symbol": "SNX9",
  "gene": "UniProtKB:Q9Y5X1",
  "term_id": "GO:0031410",
  "gene_name": "Sorting nexin-9",
  "term_label": "cytoplasmic vesicle"
}